{
  "gene_symbol": "OR5T3",
  "gene_name": "Olfactory receptor 5T3",
  "term_id": "GO:0005549",
  "term_label": "odorant binding",
  "gene": "UniProtKB:Q8NGG3"
}